{
  "term_id": "GO:0005737",
  "gene_name": "Tripartite motif-containing protein 55",
  "gene": "UniProtKB:Q9BYV6",
  "gene_symbol": "TRIM55",
  "term_label": "cytoplasm"
}